{
  "term_id": "GO:0031175",
  "term_label": "neuron projection development",
  "gene": "UniProtKB:Q8IZD0",
  "gene_name": "Sterile alpha motif domain-containing protein 14",
  "gene_symbol": "SAMD14"
}